{
  "term_label": "cytoskeleton organization",
  "term_id": "GO:0007010",
  "gene": "UniProtKB:Q7Z6J4",
  "gene_name": "FYVE, RhoGEF and PH domain-containing protein 2",
  "gene_symbol": "FGD2"
}